{
  "term_id": "GO:0008083",
  "term_label": "growth factor activity",
  "gene_symbol": "FGF16",
  "gene_name": "Fibroblast growth factor 16",
  "gene": "UniProtKB:O43320"
}